{
  "term_label": "nuclear-transcribed mRNA poly(A) tail shortening",
  "gene_symbol": "SAMD4A",
  "gene": "UniProtKB:Q9UPU9",
  "term_id": "GO:0000289",
  "gene_name": "Protein Smaug homolog 1"
}